{
  "gene_symbol": "OR10Z1",
  "gene_name": "Olfactory receptor 10Z1",
  "term_id": "GO:0005549",
  "gene": "UniProtKB:Q8NGY1",
  "term_label": "odorant binding"
}